{
  "gene_name": "Serine_threonine-protein kinase pim-3",
  "term_id": "GO:0004674",
  "gene_symbol": "PIM3",
  "gene": "UniProtKB:Q86V86",
  "term_label": "protein serine/threonine kinase activity"
}